negative regulation of TRAIL production [GO:0032719] (biological process) Definition: Any process that stops, prevents, or reduces the frequency, rate, or extent of TRAIL production. Sources: GOC:mah Also known as: down regulation of TRAIL production, down-regulation of TRAIL production, downregulation of TRAIL production, inhibition of TRAIL production, negative regulation of TRAIL biosynthetic process Relationships: is a type of regulation of TRAIL production [GO:0032679]; is a type of negative regulation of tumor necrosis factor superfamily cytokine production [GO:1903556]; RO_0002212 TRAIL production [GO:0032639]